{
  "term_id": "GO:0005634",
  "gene_symbol": "H1-4",
  "term_label": "nucleus",
  "gene": "UniProtKB:P10412",
  "gene_name": "Histone H1.4"
}